{
  "gene_symbol": "TTN",
  "term_label": "structural constituent of muscle",
  "gene_name": "Titin",
  "gene": "UniProtKB:Q8WZ42",
  "term_id": "GO:0008307"
}